{
  "term_label": "cellular response to glucocorticoid stimulus",
  "term_id": "GO:0071385",
  "gene_name": "UDP-glucuronosyltransferase 1A5",
  "gene": "UniProtKB:P35504",
  "gene_symbol": "UGT1A5"
}